{
  "term_id": "GO:0000981",
  "gene_symbol": "NEUROD2",
  "gene": "UniProtKB:Q15784",
  "term_label": "DNA-binding transcription factor activity, RNA polymerase II-specific",
  "gene_name": "Neurogenic differentiation factor 2"
}